{
  "term_id": "UNKNOWN:0003",
  "gene_name": "Coiled-coil domain-containing protein R3HCC1L",
  "term_label": "Unknown cellular component",
  "gene_symbol": "R3HCC1L",
  "gene": "UniProtKB:Q7Z5L2"
}